{
  "gene_name": "E3 ubiquitin-protein ligase RNF149",
  "gene_symbol": "RNF149",
  "gene": "UniProtKB:Q8NC42",
  "term_id": "GO:0005783",
  "term_label": "endoplasmic reticulum"
}